{
  "term_id": "GO:0045202",
  "gene": "UniProtKB:P20591",
  "term_label": "synapse",
  "gene_name": "Interferon-induced GTP-binding protein Mx1",
  "gene_symbol": "MX1"
}